{
  "gene_symbol": "DNAH10",
  "gene": "UniProtKB:Q8IVF4",
  "gene_name": "Dynein axonemal heavy chain 10",
  "term_id": "GO:0045505",
  "term_label": "dynein intermediate chain binding"
}